positive regulation of detection of mechanical stimulus involved in sensory perception of touch [GO:1905789] (BP) References: PMID:8692859 Sources: GOC:TermGenie, GO_REF:0000058 Relationships: is a type of GO:0031646; is a type of GO:0032103; is a type of regulation of detection of mechanical stimulus involved in sensory perception of touch [GO:1905787]; positively regulates detection of mechanical stimulus involved in sensory perception of touch [GO:0050976] Definition: Any process that activates or increases the frequency, rate or extent of detection of mechanical stimulus involved in sensory perception of touch. Also known as: positive regulation of perception of touch, detection of mechanical stimulus, positive regulation of perception of touch, sensory detection of mechanical stimulus, positive regulation of perception of touch, sensory transduction of mechanical stimulus, positive regulation of sensory detection of mechanical stimulus during perception of touch, positive regulation of sensory transduction of mechanical stimulus during perception of touch, positive regulation of tactition, sensory detection of mechanical stimulus, up regulation of detection of mechanical stimulus involved in sensory perception of touch, up regulation of perception of touch, detection of mechanical stimulus, up regulation of perception of touch, sensory detection of mechanical stimulus, up regulation of perception of touch, sensory transduction of mechanical stimulus, up regulation of sensory detection of mechanical stimulus during perception of touch, up regulation of sensory transduction of mechanical stimulus during perception of touch, up regulation of tactition, sensory detection of mechanical stimulus, up-regulation of detection of mechanical stimulus involved in sensory perception of touch, up-regulation of perception of touch, detection of mechanical stimulus, up-regulation of perception of touch, sensory detection of mechanical stimulus, up-regulation of perception of touch, sensory transduction of mechanical stimulus, up-regulation of sensory detection of mechanical stimulus during perception of touch, up-regulation of sensory transduction of mechanical stimulus during perception of touch, up-regulation of tactition, sensory detection of mechanical stimulus, upregulation of detection of mechanical stimulus involved in sensory perception of touch, upregulation of perception of touch, detection of mechanical stimulus, upregulation of perception of touch, sensory detection of mechanical stimulus, upregulation of perception of touch, sensory transduction of mechanical stimulus, upregulation of sensory detection of mechanical stimulus during perception of touch, upregulation of sensory transduction of mechanical stimulus during perception of touch, upregulation of tactition, sensory detection of mechanical stimulus, activation of detection of mechanical stimulus involved in sensory perception of touch, activation of perception of touch, detection of mechanical stimulus, activation of perception of touch, sensory detection of mechanical stimulus, activation of perception of touch, sensory transduction of mechanical stimulus, activation of sensory detection of mechanical stimulus during perception of touch, activation of sensory transduction of mechanical stimulus during perception of touch, activation of tactition, sensory detection of mechanical stimulus